{
  "term_label": "serine-type endopeptidase activity",
  "gene_symbol": "PLAU",
  "gene": "UniProtKB:P00749",
  "gene_name": "Urokinase-type plasminogen activator",
  "term_id": "GO:0004252"
}